(2R)-hydroxyacid dehydrogenase (quinone) activity [GO:1990464] (molecular function) Definition: Catalysis of the reaction: a (2R)-2-hydroxycarboxylate + a quinone = a 2-oxocarboxylate + a quinol. References: PMID:3013300, PMID:4582730 Sources: RHEA:11272 Also known as: D-2-hydroxyacid dehydrogenase (quinone) activity, (R)-2-hydroxy acid dehydrogenase activity, (R)-2-hydroxy-acid:(acceptor) 2-oxidoreductase activity, (R)-2-hydroxyacid:quinone oxidoreductase activity, D-lactate dehydrogenase (quinone) activity, D-lactate dehydrogenase activity, D-lactate:quinone oxidoreductase activity Note: (R)-lactate, (R)-malate and meso-tartrate are good substrates. Ubiquinone-1 and the dye 2,6-dichloroindophenol can act as acceptors; NAD+ and NADP+ are not acceptors. Relationships: is a type of oxidoreductase activity, acting on the CH-OH group of donors, quinone or similar compound as acceptor [GO:0016901]; is a type of GO:0033719 Subtypes: GO:0102029